negative regulation of epithelium regeneration [GO:1905042] (biological process) Definition: Any process that stops, prevents or reduces the frequency, rate or extent of epithelium regeneration. Also known as: down regulation of epithelium regeneration, down regulation of regeneration of epithelium, down-regulation of epithelium regeneration, down-regulation of regeneration of epithelium, downregulation of epithelium regeneration, downregulation of regeneration of epithelium, negative regulation of regeneration of epithelium, inhibition of epithelium regeneration, inhibition of regeneration of epithelium References: PMID:23221517 Sources: GOC:BHF, GOC:BHF_miRNA, GOC:TermGenie, GOC:rph, GO_REF:0000058 Relationships: is a type of negative regulation of developmental growth [GO:0048640]; is a type of regulation of epithelium regeneration [GO:1905041]; negatively regulates epithelium regeneration [GO:1990399]